{
  "gene": "UniProtKB:Q8IUF1",
  "term_label": "protein maturation",
  "gene_name": "Zinc-regulated GTPase metalloprotein activator 1B",
  "gene_symbol": "ZNG1B",
  "term_id": "GO:0051604"
}